{
  "gene_symbol": "GATC",
  "gene": "UniProtKB:O43716",
  "term_id": "GO:0032543",
  "gene_name": "Glutamyl-tRNA(Gln) amidotransferase subunit C, mitochondrial",
  "term_label": "mitochondrial translation"
}